{
  "gene": "UniProtKB:Q86UR5",
  "term_id": "GO:0098831",
  "term_label": "presynaptic active zone cytoplasmic component",
  "gene_symbol": "RIMS1",
  "gene_name": "Regulating synaptic membrane exocytosis protein 1"
}